cysteinyl leukotriene receptor binding [GO:0031745] (molecular function) Definition: Binding to a cysteinyl leukotriene receptor. Subtypes: GO:0031746, GO:0031747 Relationships: is a type of G protein-coupled receptor binding [GO:0001664] Sources: GOC:mah, GOC:nln Also known as: cysteinyl leukotriene receptor ligand